{
  "gene_symbol": "IFNK",
  "gene": "UniProtKB:Q9P0W0",
  "term_id": "GO:0006959",
  "gene_name": "Interferon kappa",
  "term_label": "humoral immune response"
}